{
  "gene": "UniProtKB:Q03181",
  "term_label": "negative regulation of transcription by RNA polymerase II",
  "gene_symbol": "PPARD",
  "term_id": "GO:0000122",
  "gene_name": "Peroxisome proliferator-activated receptor delta"
}